alanine dehydrogenase activity [GO:0000286] (molecular function) Also known as: AlaDH, L-alanine dehydrogenase activity, L-alanine:NAD+ oxidoreductase (deaminating), NAD-dependent alanine dehydrogenase activity, NAD-linked alanine dehydrogenase activity, NADH-dependent alanine dehydrogenase activity, alanine oxidoreductase activity, alpha-alanine dehydrogenase activity Definition: Catalysis of the reaction: L-alanine + H2O + NAD+ = pyruvate + NH3 + NADH + H+. Sources: EC:1.4.1.1 Relationships: is_a oxidoreductase activity, acting on the CH-NH2 group of donors [GO:0016638]